{
  "gene_name": "Keratin, type I cuticular Ha3-II",
  "term_label": "cytoskeleton",
  "gene_symbol": "KRT33B",
  "term_id": "GO:0005856",
  "gene": "UniProtKB:Q14525"
}